susceptibility to T cell mediated cytotoxicity [GO:0060370] (biological process) Definition: The process of causing a cell to become susceptible to T cell mediated cytotoxicity. Relationships: is a type of GO:0001916 Sources: GOC:dph, GOC:tb